polyprenol biosynthetic process [GO:0016094] (biological process) Also known as: polyprenol anabolism, polyprenol biosynthesis, polyprenol formation, polyprenol synthesis Relationships: is a type of GO:0008299; is a type of GO:0016093; is a type of GO:0046165 Subtypes: farnesol biosynthetic process [GO:0006715], geraniol biosynthetic process [GO:1903448] References: PMID:11108713 Sources: GOC:go_curators Definition: The chemical reactions and pathways resulting in the formation of polyprenols, prenols with more than 4 isoprenoid residues, which may be all-trans, or a mixture of cis and trans.